{
  "term_id": "GO:0005737",
  "gene_symbol": "DTD2",
  "gene_name": "D-aminoacyl-tRNA deacylase 2",
  "term_label": "cytoplasm",
  "gene": "UniProtKB:Q96FN9"
}